{
  "gene_symbol": "SEPTIN14",
  "term_id": "GO:0031105",
  "gene": "UniProtKB:Q6ZU15",
  "gene_name": "Septin-14",
  "term_label": "septin complex"
}